{
  "gene_symbol": "CXCR4",
  "term_label": "neurogenesis",
  "gene": "UniProtKB:P61073",
  "gene_name": "C-X-C chemokine receptor type 4",
  "term_id": "GO:0022008"
}